O-palmitoyltransferase activity [GO:0016416] (molecular function) Relationships: is a type of O-acyltransferase activity [GO:0008374]; is a type of GO:0016409 Definition: Catalysis of the transfer of a palmitoyl group to an oxygen atom on the acceptor molecule. Subtypes: GO:0004095, myelin-proteolipid O-palmitoyltransferase activity [GO:0047157], GO:0047965 Sources: GOC:ai